{
  "term_id": "UNKNOWN:0003",
  "term_label": "Unknown cellular component",
  "gene_symbol": "THEM6",
  "gene": "UniProtKB:Q8WUY1",
  "gene_name": "Protein THEM6"
}